glycocalyx [GO:0030112] (cellular component) Relationships: is a type of external encapsulating structure [GO:0030312] Subtypes: GO:0030114, capsule [GO:0042603], lysosomal glycocalyx [GO:0090123], stereocilium coat [GO:0120234], GO:0120238, GO:0120239, platelet glycocalyx [GO:0120240] References: PMID:28876829 Sources: GOC:krc, GOC:mlg, ISBN:0815316208 Definition: A carbohydrate rich layer at the outermost periphery of a cell.